{
  "gene": "UniProtKB:P42681",
  "gene_name": "Tyrosine-protein kinase TXK",
  "term_label": "adaptive immune response",
  "gene_symbol": "TXK",
  "term_id": "GO:0002250"
}